negative regulation of enamel mineralization [GO:0070174] (biological process) Sources: GOC:BHF, GOC:mah Relationships: is a type of negative regulation of tooth mineralization [GO:0070171]; is a type of regulation of enamel mineralization [GO:0070173]; negatively regulates GO:0070166 Definition: Any process that stops, prevents, or reduces the frequency, rate or extent of enamel mineralization, the deposition of calcium salts in tooth enamel.